{
  "term_id": "GO:0005634",
  "gene": "UniProtKB:P27695",
  "term_label": "nucleus",
  "gene_symbol": "APEX1",
  "gene_name": "DNA-(apurinic or apyrimidinic site) endonuclease"
}